ubiquitin-independent protein catabolic process via the multivesicular body sorting pathway [GO:0090611] (biological process) Definition: The chemical reactions and pathways resulting in the breakdown of a protein or peptide, via the multivesicular body (MVB) sorting pathway; proteins are sorted into MVBs, and delivered to a lysosome/vacuole for degradation. This process is independent of ubiquitination. References: PMID:22547407 Relationships: is a type of proteolysis involved in protein catabolic process [GO:0051603]; has part protein catabolic process in the vacuole [GO:0007039]; has part multivesicular body sorting pathway [GO:0071985]